{
  "term_label": "exocyst",
  "gene_name": "Tumor necrosis factor alpha-induced protein 2",
  "term_id": "GO:0000145",
  "gene": "UniProtKB:Q03169",
  "gene_symbol": "TNFAIP2"
}